{
  "gene": "UniProtKB:P22059",
  "term_label": "plasma membrane",
  "gene_symbol": "OSBP",
  "term_id": "GO:0005886",
  "gene_name": "Oxysterol-binding protein 1"
}